{
  "term_label": "cardiac muscle tissue development",
  "gene_name": "Transcription factor GATA-5",
  "term_id": "GO:0048738",
  "gene": "UniProtKB:Q9BWX5",
  "gene_symbol": "GATA5"
}